{
  "term_id": "GO:0042574",
  "gene_symbol": "RPE65",
  "term_label": "retinal metabolic process",
  "gene": "UniProtKB:Q16518",
  "gene_name": "Retinoid isomerohydrolase"
}